{
  "term_id": "GO:0005634",
  "gene_symbol": "PPEF1",
  "gene_name": "Serine_threonine-protein phosphatase with EF-hands 1",
  "gene": "UniProtKB:O14829",
  "term_label": "nucleus"
}